{
  "gene_symbol": "LAMP2",
  "gene_name": "Lysosome-associated membrane glycoprotein 2",
  "gene": "UniProtKB:P13473",
  "term_id": "GO:0009267",
  "term_label": "cellular response to starvation"
}